arginine binding [GO:0034618] (molecular function) Definition: Binding to 2-amino-5-(carbamimidamido)pentanoic acid. Sources: GOC:BHF, GOC:rl Also known as: Arg binding, aminopentanoic acid binding Relationships: is a type of amino acid binding [GO:0016597]; is a type of carboxylic acid binding [GO:0031406]; is a type of GO:0043169